negative regulation of peptide antigen transport [GO:1901040] (biological process) Also known as: down regulation of peptide antigen transport, down-regulation of peptide antigen transport, downregulation of peptide antigen transport, inhibition of peptide antigen transport Definition: Any process that stops, prevents or reduces the frequency, rate or extent of peptide antigen transport. Relationships: is a type of negative regulation of antigen processing and presentation of peptide antigen [GO:0002584]; is a type of GO:0051051; is_a regulation of peptide antigen transport [GO:1901039]; negatively regulates peptide antigen transport [GO:0046968] References: PMID:16691491 Sources: GOC:TermGenie, GOC:bf